{
  "gene_name": "Nuclear cap-binding protein subunit 3",
  "gene_symbol": "NCBP3",
  "term_id": "GO:0000339",
  "gene": "UniProtKB:Q53F19",
  "term_label": "RNA cap binding"
}